{
  "gene": "UniProtKB:A8MWA4",
  "gene_symbol": "ZNF705EP",
  "term_id": "GO:0000981",
  "gene_name": "Putative zinc finger protein 705EP",
  "term_label": "DNA-binding transcription factor activity, RNA polymerase II-specific"
}